{
  "gene_symbol": "ETFB",
  "gene": "UniProtKB:P38117",
  "gene_name": "Electron transfer flavoprotein subunit beta",
  "term_label": "electron transfer activity",
  "term_id": "GO:0009055"
}